{
  "gene_name": "C-C chemokine receptor type 8",
  "gene_symbol": "CCR8",
  "gene": "UniProtKB:P51685",
  "term_id": "GO:0019957",
  "term_label": "C-C chemokine binding"
}